{
  "term_id": "GO:0005829",
  "term_label": "cytosol",
  "gene": "UniProtKB:Q7Z6J0",
  "gene_symbol": "SH3RF1",
  "gene_name": "E3 ubiquitin-protein ligase SH3RF1"
}